{
  "term_label": "endosome",
  "term_id": "GO:0005768",
  "gene_symbol": "GPR62",
  "gene_name": "G-protein coupled receptor 62",
  "gene": "UniProtKB:Q9BZJ7"
}